structural constituent of presynaptic actin cytoskeleton [GO:0098699] (molecular function) Definition: The action of a molecule that contributes to the structural integrity of a presynaptic actin cytoskeleton. Sources: GOC:dos Relationships: is a type of structural constituent of cytoskeleton [GO:0005200]; is a type of GO:0099181; is part of presynaptic actin cytoskeleton organization [GO:0099140]; occurs in presynaptic actin cytoskeleton [GO:0099143]